{
  "term_label": "external side of plasma membrane",
  "gene_name": "Tumor necrosis factor receptor superfamily member 5",
  "gene": "UniProtKB:P25942",
  "term_id": "GO:0009897",
  "gene_symbol": "CD40"
}